cyclin binding [GO:0030332] (MF) Sources: GOC:ai Definition: Binding to cyclins, proteins whose levels in a cell varies markedly during the cell cycle, rising steadily until mitosis, then falling abruptly to zero. As cyclins reach a threshold level, they are thought to drive cells into G2 phase and thus to mitosis. Relationships: is a type of protein binding [GO:0005515]